{
  "term_label": "Unknown biological process",
  "term_id": "UNKNOWN:0002",
  "gene_name": "Exosome complex component CSL4",
  "gene": "UniProtKB:Q9Y3B2",
  "gene_symbol": "EXOSC1"
}